learned vocalization behavior [GO:0098583] (biological process) Definition: A vocalization behavior that is the result of learning. References: PMID:16418265, PMID:17035521 Sources: GOC:BHF, GOC:dos, GOC:rl Note: Examples include human speech and learned bird song. Relationships: is a type of vocalization behavior [GO:0071625]; is a type of learned vocalization behavior or vocal learning [GO:0098598]